{
  "term_label": "signaling receptor activity",
  "gene_name": "Glutamate receptor ionotropic, NMDA 1",
  "term_id": "GO:0038023",
  "gene_symbol": "GRIN1",
  "gene": "UniProtKB:Q05586"
}